{
  "gene": "UniProtKB:Q13972",
  "term_id": "GO:0007265",
  "term_label": "Ras protein signal transduction",
  "gene_symbol": "RASGRF1",
  "gene_name": "Ras-specific guanine nucleotide-releasing factor 1"
}